{
  "gene": "UniProtKB:Q8NDB2",
  "gene_name": "B-cell scaffold protein with ankyrin repeats",
  "gene_symbol": "BANK1",
  "term_label": "protein tyrosine kinase binding",
  "term_id": "GO:1990782"
}